{
  "term_id": "GO:0034098",
  "gene_name": "Ubiquitin recognition factor in ER-associated degradation protein 1",
  "gene": "UniProtKB:Q92890",
  "gene_symbol": "UFD1",
  "term_label": "VCP-NPL4-UFD1 AAA ATPase complex"
}